biochanin-A reductase activity [GO:0047706] (molecular function) Sources: EC:1.3.1.46, RHEA:12817 Also known as: dihydrobiochanin-A:NADP+ delta2-oxidoreductase activity Relationships: is_a oxidoreductase activity, acting on the CH-CH group of donors, NAD or NADP as acceptor [GO:0016628] Definition: Catalysis of the reaction: dihydrobiochanin A + NADP+ = biochanin A + H+ + NADPH.